meiotic DNA replication initiation [GO:1902974] (biological process) Relationships: is a type of nuclear cell cycle DNA replication initiation [GO:1902315]; is a type of meiotic cell cycle process [GO:1903046] Also known as: DNA replication initiation involved in meiotic DNA replication, DNA replication initiation involved in meiotic cell cycle DNA replication, initiation of meiotic DNA synthesis, initiation of premeiotic DNA replication, initiation of premeiotic DNA synthesis, premeiotic DNA replication initiation Regulation: regulated by GO:1904512; negatively regulated by negative regulation of initiation of premeiotic DNA replication [GO:1904513]; positively regulated by positive regulation of initiation of premeiotic DNA replication [GO:1904514] Definition: Any DNA replication initiation involved in meiotic cell cycle DNA replication. References: PMID:10888871 Sources: GOC:TermGenie, GO_REF:0000060